{
  "gene_name": "SPRY domain-containing SOCS box protein 4",
  "term_id": "GO:1990756",
  "gene_symbol": "SPSB4",
  "gene": "UniProtKB:Q96A44",
  "term_label": "ubiquitin-like ligase-substrate adaptor activity"
}